negative regulation of response to cytokine stimulus [GO:0060761] (biological process) Definition: Any process that decreases the rate, frequency, or extent of a response to cytokine stimulus. Subtypes: negative regulation of cytokine-mediated signaling pathway [GO:0001960], GO:0060331, negative regulation of response to macrophage colony-stimulating factor [GO:1903970] Relationships: is a type of negative regulation of response to stimulus [GO:0048585]; is a type of regulation of response to cytokine stimulus [GO:0060759]; negatively regulates response to cytokine [GO:0034097] Sources: GOC:BHF, GOC:dph, GOC:tb